{
  "gene": "UniProtKB:Q6ZN28",
  "gene_name": "Metastasis-associated in colon cancer protein 1",
  "term_id": "UNKNOWN:0001",
  "term_label": "Unknown molecular function",
  "gene_symbol": "MACC1"
}